{
  "term_label": "olfactory receptor activity",
  "gene_symbol": "OR6Y1",
  "gene_name": "Olfactory receptor 6Y1",
  "gene": "UniProtKB:Q8NGX8",
  "term_id": "GO:0004984"
}